{
  "gene_name": "Zinc finger protein 670",
  "term_label": "regulation of transcription by RNA polymerase II",
  "term_id": "GO:0006357",
  "gene": "UniProtKB:Q9BS34",
  "gene_symbol": "ZNF670"
}